{
  "term_label": "focal adhesion",
  "gene_name": "Protein PEAK3",
  "gene_symbol": "PEAK3",
  "gene": "UniProtKB:Q6ZS72",
  "term_id": "GO:0005925"
}